{
  "gene_symbol": "PIK3R6",
  "term_label": "regulation of natural killer cell mediated cytotoxicity",
  "gene_name": "Phosphoinositide 3-kinase regulatory subunit 6",
  "gene": "UniProtKB:Q5UE93",
  "term_id": "GO:0042269"
}